{
  "term_id": "GO:0005229",
  "gene_name": "Calcium-activated chloride channel regulator 2",
  "term_label": "intracellularly calcium-gated chloride channel activity",
  "gene_symbol": "CLCA2",
  "gene": "UniProtKB:Q9UQC9"
}